{
  "gene": "UniProtKB:P15018",
  "gene_symbol": "LIF",
  "term_label": "leukemia inhibitory factor receptor binding",
  "gene_name": "Leukemia inhibitory factor",
  "term_id": "GO:0005146"
}